{
  "gene_name": "Putative protein phosphatase inhibitor 2-like protein 1",
  "term_label": "protein phosphatase inhibitor activity",
  "term_id": "GO:0004864",
  "gene_symbol": "PPP1R2P1",
  "gene": "UniProtKB:Q96PQ5"
}